{
  "gene": "UniProtKB:Q7Z3U7",
  "term_label": "early endosome membrane",
  "gene_name": "Protein MON2 homolog",
  "gene_symbol": "MON2",
  "term_id": "GO:0031901"
}